{
  "term_id": "GO:0035556",
  "gene": "UniProtKB:Q9NQU5",
  "term_label": "intracellular signal transduction",
  "gene_name": "Serine_threonine-protein kinase PAK 6",
  "gene_symbol": "PAK6"
}